convergent extension involved in axis elongation [GO:0060028] (biological process) Definition: The morphogenetic process in which an epithelium narrows along one axis and lengthens in a perpendicular axis contributing to the lengthening of the axis of an organism. Regulation: regulated by regulation of convergent extension involved in axis elongation [GO:1901232]; negatively regulated by negative regulation of convergent extension involved in axis elongation [GO:1901233]; positively regulated by positive regulation of convergent extension involved in axis elongation [GO:1901234] Subtypes: convergent extension involved in somitogenesis [GO:0090246] References: PMID:12062082 Sources: GOC:dph Relationships: is a type of convergent extension [GO:0060026]; BFO_0000050 axis elongation [GO:0003401]